{
  "term_id": "GO:0032922",
  "gene": "UniProtKB:P62140",
  "term_label": "circadian regulation of gene expression",
  "gene_symbol": "PPP1CB",
  "gene_name": "Serine_threonine-protein phosphatase PP1-beta catalytic subunit"
}